{
  "term_id": "GO:0060271",
  "term_label": "cilium assembly",
  "gene_symbol": "DUSP23",
  "gene_name": "Dual specificity protein phosphatase 23",
  "gene": "UniProtKB:Q9BVJ7"
}